{
  "term_id": "GO:0060169",
  "gene_name": "Adenosine deaminase",
  "term_label": "negative regulation of adenosine receptor signaling pathway",
  "gene_symbol": "ADA",
  "gene": "UniProtKB:P00813"
}